{
  "gene_symbol": "DCHS2",
  "term_label": "cell-cell adhesion mediated by cadherin",
  "term_id": "GO:0044331",
  "gene": "UniProtKB:Q6V1P9",
  "gene_name": "Protocadherin-23"
}